tracheal outgrowth, open tracheal system [GO:0007426] (biological process) Definition: The projection of branches of an open tracheal system towards their target tissues. An example of this is found in Drosophila melanogaster. Relationships: is a type of tube morphogenesis [GO:0035239]; is part of GO:0007424 Sources: GOC:bf, GOC:mtg_sensu